{
  "gene_name": "Doublesex- and mab-3-related transcription factor 3",
  "gene_symbol": "DMRT3",
  "term_label": "adult locomotory behavior",
  "term_id": "GO:0008344",
  "gene": "UniProtKB:Q9NQL9"
}